galactosaminogalactan biosynthetic process [GO:0106218] (biological process) Definition: The chemical reactions and pathways resulting in the formation of the exopolysaccharide galactosaminogalactan. GAG is a heteropolysaccharide composed of alpha-1,4 linked galactose, N-acetyl galactosamine (GalNAc) and galactosamine (GalN). References: PMID:173713, PMID:22102815, PMID:24257745, PMID:26492565, PMID:26932183, PMID:27048799, PMID:30667338 Also known as: GAG biosynthetic process, galactosaminogalactan anabolism, galactosaminogalactan biosynthesis, galactosaminogalactan formation, galactosaminogalactan synthesis Relationships: is a type of GO:0051278